{
  "gene_symbol": "EMC2",
  "gene_name": "ER membrane protein complex subunit 2",
  "gene": "UniProtKB:Q15006",
  "term_label": "EMC complex",
  "term_id": "GO:0072546"
}